negative regulation of Wnt signaling pathway, calcium modulating pathway [GO:0045812] (biological process) Definition: Any process that stops, prevents, or reduces the frequency, rate or extent of the series of molecular signals initiated by binding of a Wnt protein to a receptor on the surface of the target cell where activated receptors leads to an increase in intracellular calcium and activation of protein kinase C (PKC). Sources: GOC:dph, GOC:go_curators, GOC:tb Also known as: down regulation of frizzled-2 signaling pathway, down-regulation of frizzled-2 signaling pathway, downregulation of frizzled-2 signaling pathway, negative regulation of Wnt receptor signaling pathway, calcium modulating pathway, negative regulation of Wnt-activated signaling pathway, calcium modulating pathway, negative regulation of frizzled-2 signaling pathway, negative regulation of frizzled-2 signalling pathway, inhibition of frizzled-2 signaling pathway Relationships: is a type of GO:0008591; is_a GO:2000051; negatively regulates Wnt signaling pathway, calcium modulating pathway [GO:0007223]